dendritic spine membrane [GO:0032591] (cellular component) Sources: GOC:mah Relationships: is a type of neuron projection membrane [GO:0032589]; is a type of GO:0097060; is part of GO:0032590; is part of GO:0043197 Definition: The portion of the plasma membrane surrounding a dendritic spine.